{
  "term_id": "UNKNOWN:0001",
  "gene_symbol": "MSL3B",
  "term_label": "Unknown molecular function",
  "gene": "UniProtKB:P0C860",
  "gene_name": "Putative male-specific lethal-3 protein-like 2"
}